{
  "gene_name": "Ubiquitin carboxyl-terminal hydrolase 17-like protein 10",
  "term_id": "GO:0031647",
  "gene_symbol": "USP17L10",
  "term_label": "regulation of protein stability",
  "gene": "UniProtKB:C9JJH3"
}